{
  "term_label": "Unknown molecular function",
  "term_id": "UNKNOWN:0001",
  "gene_symbol": "VSTM4",
  "gene_name": "V-set and transmembrane domain-containing protein 4",
  "gene": "UniProtKB:Q8IW00"
}